anthranilate synthase activity [GO:0004049] (molecular function) Definition: Catalysis of the reaction: chorismate + L-glutamine = anthranilate + pyruvate + L-glutamate. Also known as: anthranilate synthetase activity, chorismate pyruvate-lyase (amino-accepting) activity Relationships: is_a GO:0016833 Sources: EC:4.1.3.27